steroid 7-alpha-hydroxylase activity [GO:0008387] (molecular function) Also known as: cytochrome P450 CYP2A12 Subtypes: GO:0008123, oxysterol 7-alpha-hydroxylase activity [GO:0008396], 24S-hydroxycholesterol 7-alpha-hydroxylase activity [GO:0033782], 25-hydroxycholesterol 7-alpha-hydroxylase activity [GO:0033783] Definition: Catalysis of the reaction: a steroid + AH2 + O2 = 7-alpha-hydroxysteroid + H2O. Relationships: is a type of steroid hydroxylase activity [GO:0008395]; is_a oxidoreductase activity, acting on paired donors, with incorporation or reduction of molecular oxygen [GO:0016705] Sources: GOC:mah